{
  "gene": "UniProtKB:O95989",
  "term_id": "GO:0071543",
  "gene_symbol": "NUDT3",
  "gene_name": "Diphosphoinositol polyphosphate phosphohydrolase 1",
  "term_label": "diphosphoinositol polyphosphate metabolic process"
}